{
  "term_id": "GO:0015012",
  "gene_name": "Bifunctional heparan sulfate N-deacetylase_N-sulfotransferase 1",
  "gene": "UniProtKB:P52848",
  "gene_symbol": "NDST1",
  "term_label": "heparan sulfate proteoglycan biosynthetic process"
}